{
  "gene_symbol": "CA9",
  "term_label": "Unknown biological process",
  "gene_name": "Carbonic anhydrase 9",
  "term_id": "UNKNOWN:0002",
  "gene": "UniProtKB:Q16790"
}